{
  "gene_name": "Sodium_potassium-transporting ATPase subunit beta-1-interacting protein 3",
  "term_label": "Unknown molecular function",
  "gene_symbol": "NKAIN3",
  "term_id": "UNKNOWN:0001",
  "gene": "UniProtKB:Q8N8D7"
}